{
  "term_label": "Unknown biological process",
  "gene_symbol": "ZCCHC2",
  "gene": "UniProtKB:Q9C0B9",
  "gene_name": "Zinc finger CCHC domain-containing protein 2",
  "term_id": "UNKNOWN:0002"
}